{
  "term_id": "GO:0017017",
  "gene_symbol": "DUSP9",
  "gene": "UniProtKB:Q99956",
  "term_label": "MAP kinase tyrosine/serine/threonine phosphatase activity",
  "gene_name": "Dual specificity protein phosphatase 9"
}